ephedrine dehydrogenase activity [GO:0047877] (molecular function) Relationships: is a type of oxidoreductase activity, acting on the CH-NH group of donors, NAD or NADP as acceptor [GO:0016646] Definition: Catalysis of the reaction: (1R,2S)-ephedrine + NAD+ = (R)-2-methylimino-1-phenylpropan-1-ol + 2 H+ + NADH. Sources: EC:1.5.1.18, RHEA:16289 Also known as: (-)-ephedrine:NAD+ 2-oxidoreductase activity